{
  "term_label": "anterior/posterior pattern specification",
  "gene": "UniProtKB:Q9NQ87",
  "term_id": "GO:0009952",
  "gene_name": "Hairy_enhancer-of-split related with YRPW motif-like protein",
  "gene_symbol": "HEYL"
}